{
  "gene": "UniProtKB:P49459",
  "gene_symbol": "UBE2A",
  "term_id": "GO:0000209",
  "gene_name": "Ubiquitin-conjugating enzyme E2 A",
  "term_label": "protein polyubiquitination"
}